{
  "term_id": "UNKNOWN:0002",
  "gene": "UniProtKB:A0A8Q3SIG1",
  "gene_symbol": "LOC400499",
  "gene_name": "Vitellogenin domain-containing protein",
  "term_label": "Unknown biological process"
}